{
  "gene_name": "Protein LSM14 homolog A",
  "term_label": "P-body",
  "gene_symbol": "LSM14A",
  "gene": "UniProtKB:Q8ND56",
  "term_id": "GO:0000932"
}